{
  "gene_symbol": "FGFR1OP2",
  "term_id": "UNKNOWN:0003",
  "gene_name": "FGFR1 oncogene partner 2",
  "gene": "UniProtKB:Q9NVK5",
  "term_label": "Unknown cellular component"
}